{
  "gene": "UniProtKB:Q14677",
  "term_id": "GO:0006897",
  "gene_name": "Clathrin interactor 1",
  "gene_symbol": "CLINT1",
  "term_label": "endocytosis"
}